{
  "gene_name": "Inositol-trisphosphate 3-kinase B",
  "term_label": "cytoplasm",
  "gene": "UniProtKB:P27987",
  "term_id": "GO:0005737",
  "gene_symbol": "ITPKB"
}